{
  "gene_name": "Zinc finger protein 672",
  "term_id": "GO:0005634",
  "gene_symbol": "ZNF672",
  "gene": "UniProtKB:Q499Z4",
  "term_label": "nucleus"
}